regulation of timing of meristematic phase transition [GO:0048506] (BP) Definition: Any process that modulates the rate, frequency or extent of a change in identity of a meristem at a characteristic predetermined time point. Sources: GOC:dph, GOC:jid, GOC:tb Relationships: is a type of regulation of development, heterochronic [GO:0040034]; is a type of regulation of meristem development [GO:0048509] Subtypes: GO:0048510